{
  "gene_name": "Arginine-hydroxylase NDUFAF5, mitochondrial",
  "gene_symbol": "NDUFAF5",
  "gene": "UniProtKB:Q5TEU4",
  "term_label": "mitochondrial respiratory chain complex I assembly",
  "term_id": "GO:0032981"
}